negative regulation of dendritic cell antigen processing and presentation [GO:0002605] (biological process) Subtypes: GO:0002608, GO:0002611 Relationships: is a type of negative regulation of antigen processing and presentation [GO:0002578]; is a type of regulation of dendritic cell antigen processing and presentation [GO:0002604]; RO_0002212 dendritic cell antigen processing and presentation [GO:0002468] Sources: GOC:add Definition: Any process that stops, prevents, or reduces the frequency, rate, or extent of dendritic cell antigen processing and presentation. Also known as: down regulation of dendritic cell antigen processing and presentation, down-regulation of dendritic cell antigen processing and presentation, downregulation of dendritic cell antigen processing and presentation, inhibition of dendritic cell antigen processing and presentation